{
  "term_id": "GO:0048040",
  "term_label": "UDP-glucuronate decarboxylase activity",
  "gene_symbol": "UXS1",
  "gene": "UniProtKB:Q8NBZ7",
  "gene_name": "UDP-glucuronic acid decarboxylase 1"
}